hard palate development [GO:0060022] (biological process) Also known as: palatum durum development Definition: The biological process whose specific outcome is the progression of the hard palate from an initial condition to its mature state. This process begins with the formation of the structure and ends with the mature structure, whatever form that may be including its natural destruction. The hard palate is the anterior portion of the palate consisting of bone and mucous membranes. Sources: GOC:dph, ISBN:0721662544 Relationships: is a type of anatomical structure development [GO:0048856]; BFO_0000050 secondary palate development [GO:0062009]